floor plate morphogenesis [GO:0033505] (biological process) Sources: GOC:dh Relationships: is a type of embryonic morphogenesis [GO:0048598]; is a type of GO:0048729; BFO_0000050 floor plate development [GO:0033504] Definition: The process in which the anatomical structure of the floor plate is generated and organized.